{
  "gene": "UniProtKB:Q86WK9",
  "term_id": "GO:0005496",
  "gene_name": "Membrane progestin receptor alpha",
  "term_label": "steroid binding",
  "gene_symbol": "PAQR7"
}